{
  "gene_name": "Transmembrane protein 42",
  "gene_symbol": "TMEM42",
  "term_label": "Unknown molecular function",
  "gene": "UniProtKB:Q69YG0",
  "term_id": "UNKNOWN:0001"
}